{
  "gene": "UniProtKB:Q9ULJ8",
  "gene_symbol": "PPP1R9A",
  "term_label": "cytoplasm",
  "gene_name": "Neurabin-1",
  "term_id": "GO:0005737"
}